{
  "gene_name": "Medium-wave-sensitive opsin 2",
  "term_id": "GO:0007186",
  "gene": "UniProtKB:P0DN77",
  "gene_symbol": "OPN1MW2",
  "term_label": "G protein-coupled receptor signaling pathway"
}